{
  "gene_name": "Nuclear receptor-binding protein",
  "gene_symbol": "NRBP1",
  "term_label": "protein serine/threonine kinase activity",
  "term_id": "GO:0004674",
  "gene": "UniProtKB:Q9UHY1"
}